transport of virus in host, cell to cell [GO:0046740] (biological process) Definition: The transport of a virus between adjacent cells in a multicellular organism. Sources: GOC:bf, GOC:jl, ISBN:0781718325 Also known as: cell to cell spread of virus within host, intercellular virus transport, spread of virus within host, cell to cell, viral spread within host, cell to cell, spread of virus in host, cell to cell Relationships: is a type of transport of virus in multicellular host [GO:0046739]